Cul3-RING ubiquitin ligase complex [GO:0031463] (cellular component) References: PMID:15571813, PMID:15688063 Relationships: is a type of GO:0031461 Definition: A ubiquitin ligase complex in which a cullin from the Cul3 subfamily and a RING domain protein form the catalytic core; substrate specificity is conferred by a BTB-domain-containing protein. Also known as: BC3B complex, BCR3 complex, CDL3 complex, CRL3 complex, cullin-RING ligase 3, SCF3 complex